{
  "gene_name": "T-cell surface glycoprotein CD8 beta-2 chain",
  "term_id": "UNKNOWN:0002",
  "term_label": "Unknown biological process",
  "gene_symbol": "CD8B2",
  "gene": "UniProtKB:A6NJW9"
}